{
  "term_label": "cytoplasm",
  "gene_symbol": "HLCS",
  "gene": "UniProtKB:P50747",
  "gene_name": "Biotin--protein ligase",
  "term_id": "GO:0005737"
}